glycoprotein metabolic process [GO:0009100] (biological process) Relationships: is a type of protein metabolic process [GO:0019538]; is a type of carbohydrate derivative metabolic process [GO:1901135] Regulation: regulated by modulation by host of viral glycoprotein metabolic process [GO:0044870]; regulated by GO:1903018; negatively regulated by negative regulation of glycoprotein metabolic process [GO:1903019]; positively regulated by positive regulation of glycoprotein metabolic process [GO:1903020] Definition: The chemical reactions and pathways involving glycoproteins, a protein that contains covalently bound glycose (i.e. monosaccharide) residues; the glycose occurs most commonly as oligosaccharide or fairly small polysaccharide but occasionally as monosaccharide. Also known as: glycoprotein metabolism Sources: GOC:go_curators, ISBN:0198506732 Subtypes: proteoglycan metabolic process [GO:0006029], glycoprotein catabolic process [GO:0006516], protein deglycosylation [GO:0006517], glycoprotein biosynthetic process [GO:0009101], elastin metabolic process [GO:0051541]